{
  "term_label": "triglyceride homeostasis",
  "gene_symbol": "APOC3",
  "gene_name": "Apolipoprotein C-III",
  "gene": "UniProtKB:P02656",
  "term_id": "GO:0070328"
}